embryonic skeletal system morphogenesis [GO:0048704] (biological process) Also known as: embryonic skeletal morphogenesis Definition: The process in which the anatomical structures of the skeleton are generated and organized during the embryonic phase. Subtypes: GO:0048701, GO:0060272 References: PMID:16049113 Sources: GOC:dph, GOC:dsf, GOC:jid, GOC:tb Relationships: is a type of embryonic organ morphogenesis [GO:0048562]; is a type of GO:0048705; BFO_0000050 embryonic skeletal system development [GO:0048706]